GTP cyclohydrolase binding [GO:0044549] (molecular function) Definition: Binding to a GTP cyclohydrolase. Sources: GOC:jl Also known as: GTP cyclohydrolase I binding Relationships: is a type of GO:0019899